{
  "gene": "UniProtKB:O95025",
  "term_label": "plasma membrane",
  "gene_symbol": "SEMA3D",
  "gene_name": "Semaphorin-3D",
  "term_id": "GO:0005886"
}